{
  "gene_name": "Twinfilin-1",
  "term_id": "GO:0030016",
  "gene_symbol": "TWF1",
  "gene": "UniProtKB:Q12792",
  "term_label": "myofibril"
}